{
  "gene": "UniProtKB:O15321",
  "gene_name": "Transmembrane 9 superfamily member 1",
  "term_label": "membrane",
  "gene_symbol": "TM9SF1",
  "term_id": "GO:0016020"
}